{
  "gene": "UniProtKB:P80075",
  "gene_name": "C-C motif chemokine 8",
  "term_id": "GO:0048245",
  "term_label": "eosinophil chemotaxis",
  "gene_symbol": "CCL8"
}